{
  "gene": "UniProtKB:Q30KP8",
  "gene_symbol": "DEFB136",
  "term_id": "GO:0001530",
  "term_label": "lipopolysaccharide binding",
  "gene_name": "Defensin beta 136"
}